protein N-linked glycosylation [GO:0006487] (biological process) Definition: A protein glycosylation process in which a carbohydrate or carbohydrate derivative unit is added to a protein via the N4 atom of an asparagine residue. References: PMID:35536965 Also known as: protein amino acid N-linked glycosylation, N-glycan biosynthesis, N-glycan metabolism Relationships: is a type of glycoprotein biosynthetic process [GO:0009101] Subtypes: GO:0018279, GO:0140263